{
  "gene_name": "Zinc finger protein 639",
  "gene": "UniProtKB:Q9UID6",
  "gene_symbol": "ZNF639",
  "term_label": "DNA-binding transcription factor activity",
  "term_id": "GO:0003700"
}